{
  "gene_name": "Synaptotagmin-5",
  "term_label": "SNARE binding",
  "gene_symbol": "SYT5",
  "term_id": "GO:0000149",
  "gene": "UniProtKB:O00445"
}